{
  "gene_name": "Zinc finger protein 37A",
  "term_label": "RNA polymerase II cis-regulatory region sequence-specific DNA binding",
  "gene_symbol": "ZNF37A",
  "term_id": "GO:0000978",
  "gene": "UniProtKB:P17032"
}